{
  "term_label": "cytoplasm",
  "gene_symbol": "RITA1",
  "gene": "UniProtKB:Q96K30",
  "term_id": "GO:0005737",
  "gene_name": "RBPJ-interacting and tubulin-associated protein 1"
}